{
  "gene_name": "Olfactory receptor 8D4",
  "term_label": "sensory perception of smell",
  "gene": "UniProtKB:Q8NGM9",
  "term_id": "GO:0007608",
  "gene_symbol": "OR8D4"
}